{
  "gene_symbol": "UNQ6190_PRO20217",
  "gene": "UniProtKB:Q6UXQ8",
  "term_label": "Unknown biological process",
  "gene_name": "Putative uncharacterized protein UNQ6190_PRO20217",
  "term_id": "UNKNOWN:0002"
}